gel phase of interstitial matrix [GO:0140150] (cellular component) Definition: Hydrogel filling the interstitial extracellular matrix space. Composed of proteoglycans such as hyaluronan and lectin-binding proteoglycans, SPOCK proteoglycans and small leucin-rich proteoglycan (SLRP). References: PMID:21123617, PMID:25701227, PMID:33605520, PMID:39223427 Relationships: is a type of GO:0030312; is part of GO:0005614